acylglycerone-phosphate reductase (NADP+) activity [GO:0000140] (molecular function) Also known as: 1-acyldihydroxyacetone-phosphate reductase activity, 1-palmitoylglycerol-3-phosphate:NADP+ oxidoreductase activity, acyldihydroxyacetone phosphate reductase activity, palmitoyl dihydroxyacetone phosphate reductase activity, palmitoyl-dihydroxyacetone-phosphate reductase activity, palmitoyldihydroxyacetone-phosphate reductase activity Sources: RHEA:17341 Relationships: is a type of oxidoreductase activity, acting on the CH-OH group of donors, NAD or NADP as acceptor [GO:0016616] Definition: Catalysis of the reaction: 1-hexadecanoyl-sn-glycero-3-phosphate + NADP+ = 1-hexadecanoylglycerone 3-phosphate + H+ + NADPH.